{
  "gene_name": "Nurim",
  "term_id": "UNKNOWN:0001",
  "term_label": "Unknown molecular function",
  "gene": "UniProtKB:Q8IXM6",
  "gene_symbol": "NRM"
}